{
  "gene": "UniProtKB:Q9BYG4",
  "term_id": "GO:0007163",
  "term_label": "establishment or maintenance of cell polarity",
  "gene_name": "Partitioning defective 6 homolog gamma",
  "gene_symbol": "PARD6G"
}